insulin receptor complex [GO:0005899] (cellular component) Relationships: is a type of plasma membrane signaling receptor complex [GO:0098802]; is a type of protein kinase complex [GO:1902911] Sources: ISBN:0198506732 Definition: A disulfide-bonded, heterotetrameric receptor complex. The alpha chains are entirely extracellular, while each beta chain has one transmembrane domain. The ligand binds to the alpha subunit extracellular domain and the kinase is associated with the beta subunit intracellular domain.